{
  "gene": "UniProtKB:P54840",
  "term_label": "cytoplasm",
  "term_id": "GO:0005737",
  "gene_symbol": "GYS2",
  "gene_name": "Glycogen [starch] synthase, liver"
}